{
  "gene": "UniProtKB:Q7Z7M1",
  "term_label": "G protein-coupled receptor signaling pathway",
  "gene_name": "Adhesion G-protein coupled receptor D2",
  "term_id": "GO:0007186",
  "gene_symbol": "ADGRD2"
}